{
  "gene_symbol": "FBF1",
  "gene": "UniProtKB:Q8TES7",
  "term_id": "GO:0005814",
  "term_label": "centriole",
  "gene_name": "Fas-binding factor 1"
}